retrotransposition [GO:0032197] (biological process) Regulation: negatively regulated by GO:0010526 Definition: A type of transposition in which a transposable element (transposon) copies and pastes itself into a different genomic location by transcription and convertsion of the transcribed RNA back into DNA through reverse transcription. References: PMID:26912865, PMID:30416149, PMID:30958115, PMID:32588192 Sources: ISBN:1555812090 Relationships: is a type of transposition [GO:0032196] Also known as: Class I transposition, RNA-mediated transposition, retrotransposon transposition, transposition via RNA intermediate, transposition, RNA-mediated, Tf transposition, Ty element transposition, Ty1 element transposition, Ty2 element transposition, Ty3 element transposition